{
  "term_id": "GO:0005737",
  "gene_symbol": "LIN28B",
  "gene_name": "Protein lin-28 homolog B",
  "gene": "UniProtKB:Q6ZN17",
  "term_label": "cytoplasm"
}